{
  "gene_name": "Ephrin-B2",
  "term_label": "ephrin receptor binding",
  "gene_symbol": "EFNB2",
  "term_id": "GO:0046875",
  "gene": "UniProtKB:P52799"
}